3'-phosphoadenosine 5'-phosphosulfate transport [GO:0046963] (biological process) Also known as: 3'-phosphoadenosine 5'-phosphosulphate transport, PAPS transport, adenosine 3'-phosphate 5'-phosphosulfate transport Relationships: is a type of organic anion transport [GO:0015711]; is a type of purine ribonucleotide transport [GO:0015868]; is a type of adenine nucleotide transport [GO:0051503]; is a type of sulfur compound transport [GO:0072348] Subtypes: GO:1902559 Sources: ISBN:0198506732 Definition: The directed movement of 3'-phosphoadenosine 5'-phosphosulfate, a naturally occurring mixed anhydride synthesized from adenosine 5'-phosphosulfate, into, out of or within a cell, or between cells, by means of some agent such as a transporter or pore.